{
  "gene_name": "Secretagogin",
  "term_id": "GO:0045202",
  "gene": "UniProtKB:O76038",
  "gene_symbol": "SCGN",
  "term_label": "synapse"
}